meiotic spindle midzone [GO:1990385] (cellular component) References: PMID:12707312 Sources: GOC:kmv Relationships: is a type of GO:0051233; is part of meiotic spindle [GO:0072687] Definition: The area in the center of the meiotic spindle where the spindle microtubules from opposite poles overlap.